cellular component biogenesis [GO:0044085] (biological process) Regulation: regulated by regulation of cellular component biogenesis [GO:0044087]; positively regulated by positive regulation of cellular component biogenesis [GO:0044089] Relationships: is_a GO:0071840 Subtypes: seed oilbody biogenesis [GO:0010344], nucleologenesis [GO:0017126], ribonucleoprotein complex biogenesis [GO:0022613], primary cell septum biogenesis [GO:0031671], cell wall biogenesis [GO:0042546], membrane biogenesis [GO:0044091], GO:0061110, extracellular vesicle biogenesis [GO:0140112], secondary cell septum biogenesis [GO:1990344] Sources: GOC:jl, GOC:mah Definition: A process that results in the biosynthesis of constituent macromolecules, assembly, and arrangement of constituent parts of a cellular component. Includes biosynthesis of constituent macromolecules, and those macromolecular modifications that are involved in synthesis or assembly of the cellular component. Also known as: cellular component biogenesis at cellular level